homogentisate solanesyltransferase activity [GO:0010357] (MF) Relationships: is a type of GO:0010354 Also known as: HST activity, homogentisate solanyltransferase activity References: PMID:16989822 Sources: RHEA:37995 Definition: Catalysis of the reaction: all-trans-nonaprenyl diphosphate + H+ + homogentisate = 2-methyl-6-all-trans-nonaprenylbenzene-1,4-diol + CO2 + diphosphate. 2-methyl-6-solanyl-1,4-benzoquinonone is also known as 2-methyl-6-solanesylplastoquinol and all-trans-nonaprenyl diphosphate as solanesyl diphosphate.